thiazole biosynthetic process [GO:0052837] (biological process) Also known as: thiazole anabolism, thiazole biosynthesis, thiazole formation, thiazole synthesis Sources: GOC:curators Definition: The chemical reactions and pathways resulting in the formation of a thiazole, a five-membered heterocyclic ring structure containing a sulfur in the 1-position and a nitrogen in the 3-position. Relationships: is a type of sulfur compound biosynthetic process [GO:0044272]; is a type of thiazole metabolic process [GO:0052838]